anastral spindle assembly involved in male meiosis [GO:0009971] (biological process) Definition: The aggregation, arrangement and bonding together of a set of components to form the anastral spindle in male meiotic cells. References: PMID:11973272 Sources: GOC:tb Relationships: is a type of spindle assembly involved in male meiosis [GO:0007053]; is a type of GO:0055048